positive regulation of dehydroepiandrosterone secretion [GO:2000842] (biological process) Sources: GOC:sl Also known as: positive regulation of 3beta-hydroxyandrost-5-en-17-one secretion, positive regulation of DHEA secretion, positive regulation of dehydroisoandrosterone secretion Relationships: is a type of GO:0032370; is a type of positive regulation of hormone secretion [GO:0046887]; is a type of GO:2000840; positively regulates GO:0035942 Definition: Any process that activates or increases the frequency, rate or extent of dehydroepiandrosterone secretion.